{
  "gene_symbol": "GAGE2A",
  "term_label": "Unknown biological process",
  "term_id": "UNKNOWN:0002",
  "gene_name": "G antigen 2A",
  "gene": "UniProtKB:Q6NT46"
}